{
  "gene_name": "Mesoderm induction early response protein 2",
  "gene": "UniProtKB:Q8N344",
  "gene_symbol": "MIER2",
  "term_label": "negative regulation of transcription by RNA polymerase II",
  "term_id": "GO:0000122"
}